{
  "gene_name": "Cobalamin binding intrinsic factor",
  "gene_symbol": "CBLIF",
  "term_label": "extracellular space",
  "term_id": "GO:0005615",
  "gene": "UniProtKB:P27352"
}